{
  "term_label": "Unknown cellular component",
  "gene": "UniProtKB:Q495M9",
  "gene_symbol": "USH1G",
  "term_id": "UNKNOWN:0003",
  "gene_name": "pre-mRNA splicing regulator USH1G"
}